{
  "gene_name": "Histone H2A-Bbd type 2_3",
  "gene_symbol": "H2AB3",
  "gene": "UniProtKB:P0C5Z0",
  "term_id": "GO:0005634",
  "term_label": "nucleus"
}